{
  "gene_name": "Transmembrane protein 71",
  "term_id": "UNKNOWN:0001",
  "gene_symbol": "TMEM71",
  "term_label": "Unknown molecular function",
  "gene": "UniProtKB:Q6P5X7"
}